antigen processing and presentation initiated by pattern recognition receptor mediated uptake of antigen [GO:0002748] (BP) Sources: GOC:add, ISBN:0781735149 Also known as: antigen processing and presentation initiated by PAMP receptor mediated uptake of antigen, antigen processing and presentation initiated by PRR mediated uptake of antigen Relationships: is a type of antigen processing and presentation initiated by receptor mediated uptake of antigen [GO:0002745] Definition: Antigen processing and presentation which is initiated by uptake of antigen bound to a cell surface pattern recognition receptor (PRR).